{
  "gene_symbol": "PHLDA1",
  "term_id": "GO:0005634",
  "gene_name": "Pleckstrin homology-like domain family A member 1",
  "gene": "UniProtKB:Q8WV24",
  "term_label": "nucleus"
}